microglial cell activation involved in immune response [GO:0002282] (biological process) Definition: The change in morphology and behavior of a microglial cell resulting from exposure to a cytokine, chemokine, cellular ligand, or soluble factor, leading to the initiation or perpetuation of an immune response. Sources: GOC:add, ISBN:0781735149 Relationships: is a type of GO:0001774; is a type of GO:0002281 Also known as: microglial cell activation during immune response